{
  "gene_name": "HLA class I histocompatibility antigen, alpha chain F",
  "gene": "UniProtKB:P30511",
  "term_label": "signaling receptor binding",
  "gene_symbol": "HLA-F",
  "term_id": "GO:0005102"
}